retrograde trans-synaptic signaling by nitric oxide, modulating synaptic transmission [GO:0098925] (biological process) Relationships: is a type of retrograde trans-synaptic signaling by nitric oxide [GO:0098924]; is a type of trans-synaptic signaling by nitric oxide, modulating synaptic transmission [GO:0099555] Sources: GOC:dos Note: Note that this term was created for the SynGO project, and will be obsoleted when the SynGO annotations are made in Noctua. Definition: Modulation of synaptic transmission by cell-cell signaling from postsynapse to presynapse, across the synaptic cleft, mediated by nitric oxide.